{
  "term_label": "execution phase of apoptosis",
  "gene": "UniProtKB:P42574",
  "term_id": "GO:0097194",
  "gene_symbol": "CASP3",
  "gene_name": "Caspase-3"
}